{
  "gene": "UniProtKB:O95782",
  "gene_symbol": "AP2A1",
  "term_id": "GO:0035615",
  "term_label": "clathrin adaptor activity",
  "gene_name": "AP-2 complex subunit alpha-1"
}